COPII receptor activity [GO:0097020] (molecular function) Definition: Binding specifically to a substance (cargo) to deliver it to a COPII transport vesicle. Cargo receptors span a membrane (either the plasma membrane or a vesicle membrane), binding simultaneously to cargo molecules and coat adaptors, to efficiently recruit soluble proteins to nascent vesicles. Relationships: is a type of cargo receptor activity [GO:0038024] References: PMID:16957051, PMID:20236934 Sources: GOC:rb